{
  "gene": "UniProtKB:Q9NRZ7",
  "gene_name": "1-acyl-sn-glycerol-3-phosphate acyltransferase gamma",
  "term_id": "GO:0012505",
  "gene_symbol": "AGPAT3",
  "term_label": "endomembrane system"
}